basophil chemotaxis [GO:0002575] (biological process) Definition: The movement of a basophil in response to an external stimulus. References: PMID:11292027 Sources: GOC:add Relationships: is a type of granulocyte chemotaxis [GO:0071621]